cyanamide hydratase activity [GO:0018820] (molecular function) Also known as: urea hydro-lyase (cyanamide-forming), urea hydro-lyase activity Sources: EC:4.2.1.69, RHEA:23056 Definition: Catalysis of the reaction: urea = cyanamide + H2O. Relationships: is a type of GO:0016836